{
  "term_id": "GO:0042073",
  "gene_name": "Intraflagellar transport protein 172 homolog",
  "gene_symbol": "IFT172",
  "term_label": "intraciliary transport",
  "gene": "UniProtKB:Q9UG01"
}